{
  "gene_name": "AMSH-like protease",
  "term_label": "endosome",
  "gene": "UniProtKB:Q96FJ0",
  "gene_symbol": "STAMBPL1",
  "term_id": "GO:0005768"
}